{
  "term_id": "GO:0043542",
  "term_label": "endothelial cell migration",
  "gene_symbol": "TGFB1I1",
  "gene": "UniProtKB:O43294",
  "gene_name": "Transforming growth factor beta-1-induced transcript 1 protein"
}